CCR6 chemokine receptor binding [GO:0031731] (molecular function) Definition: Binding to a CCR6 chemokine receptor. Relationships: is a type of CCR chemokine receptor binding [GO:0048020] Also known as: LARC receptor binding, CCR6 chemokine receptor ligand Sources: GOC:mah, GOC:nln